{
  "gene_name": "Acetyl-CoA carboxylase 2",
  "term_label": "acetyl-CoA carboxylase activity",
  "gene_symbol": "ACACB",
  "term_id": "GO:0003989",
  "gene": "UniProtKB:O00763"
}